{
  "term_label": "signal transduction",
  "gene_name": "Olfactory receptor 1J4",
  "gene": "UniProtKB:Q8NGS1",
  "term_id": "GO:0007165",
  "gene_symbol": "OR1J4"
}